cellular response to indolebutyric acid stimulus [GO:0071366] (biological process) Also known as: cellular response to IBA stimulus, cellular response to indole-3-butyric acid stimulus Definition: Any process that results in a change in state or activity of a cell (in terms of movement, secretion, enzyme production, gene expression, etc.) as a result of an indolebutyric acid stimulus. Sources: GOC:mah Relationships: is a type of GO:0071365; is a type of response to indolebutyric acid [GO:0080026]; is a type of cellular response to nitrogen compound [GO:1901699]; is_a GO:1901701